{
  "term_label": "Unknown cellular component",
  "gene_name": "Putative STAG3-like protein 1",
  "gene": "UniProtKB:P0CL83",
  "term_id": "UNKNOWN:0003",
  "gene_symbol": "STAG3L1"
}